vulval cell fate specification [GO:0072327] (biological process) References: PMID:11236714 Sources: GOC:kmv, GOC:mah, ISBN:087969307X Definition: The process in which a cell becomes capable of differentiating autonomously into a nematode vulval cell in an environment that is neutral with respect to the developmental pathway; upon specification, the cell fate can be reversed. In nematodes, the vulva is formed from ventral epidermal cells during larval stages to give rise to a fully formed adult vulva, which is the egg-laying organ of female and hermaphrodite nematodes. Relationships: is a type of cell fate specification [GO:0001708]; BFO_0000050 vulval cell fate commitment [GO:0072325]